{
  "gene": "UniProtKB:Q5GLZ8",
  "term_id": "GO:0006511",
  "term_label": "ubiquitin-dependent protein catabolic process",
  "gene_symbol": "HERC4",
  "gene_name": "Probable E3 ubiquitin-protein ligase HERC4"
}